{
  "term_id": "GO:0007167",
  "term_label": "enzyme-linked receptor protein signaling pathway",
  "gene_name": "GRB2-related adapter protein-like",
  "gene_symbol": "GRAPL",
  "gene": "UniProtKB:Q8TC17"
}